optical nerve axon regeneration [GO:0101027] (biological process) References: PMID:16699509 Sources: GOC:pga Definition: The regrowth of axons of the optical nerve following their loss or damage. Regulation: RO_0002211 by GO:1905591; negatively regulated by GO:1905592; RO_0002213 by positive regulation of optical nerve axon regeneration [GO:1905593] Relationships: is a type of axon regeneration [GO:0031103]